{
  "gene_symbol": "HM13",
  "term_id": "GO:0098553",
  "gene_name": "Minor histocompatibility antigen H13",
  "term_label": "lumenal side of endoplasmic reticulum membrane",
  "gene": "UniProtKB:Q8TCT9"
}